{
  "term_id": "GO:0006886",
  "gene_name": "Ras-related protein Rab-28",
  "term_label": "intracellular protein transport",
  "gene": "UniProtKB:P51157",
  "gene_symbol": "RAB28"
}